{
  "term_id": "GO:0004984",
  "gene_name": "Olfactory receptor 51F1",
  "term_label": "olfactory receptor activity",
  "gene_symbol": "OR51F1",
  "gene": "UniProtKB:A6NGY5"
}